{
  "term_id": "GO:0008260",
  "gene_name": "Succinyl-CoA:3-ketoacid coenzyme A transferase 2, mitochondrial",
  "gene": "UniProtKB:Q9BYC2",
  "gene_symbol": "OXCT2",
  "term_label": "succinyl-CoA:3-oxo-acid CoA-transferase activity"
}